{
  "gene_name": "ATPase GET3",
  "term_label": "tail-anchored membrane protein insertion into ER membrane",
  "gene_symbol": "GET3",
  "term_id": "GO:0071816",
  "gene": "UniProtKB:O43681"
}